{
  "gene_name": "Serpin B7",
  "gene_symbol": "SERPINB7",
  "term_id": "UNKNOWN:0002",
  "term_label": "Unknown biological process",
  "gene": "UniProtKB:O75635"
}